{
  "gene_symbol": "NRCAM",
  "gene_name": "Neuronal cell adhesion molecule",
  "term_id": "GO:0007420",
  "gene": "UniProtKB:Q92823",
  "term_label": "brain development"
}